{
  "term_id": "GO:0000981",
  "gene": "UniProtKB:Q8TF47",
  "gene_symbol": "ZFP90",
  "gene_name": "Zinc finger protein 90 homolog",
  "term_label": "DNA-binding transcription factor activity, RNA polymerase II-specific"
}